female germ cell nucleus [GO:0001674] (cellular component) Subtypes: germinal vesicle [GO:0042585] Definition: The nucleus of the female germ cell, a reproductive cell in females. Sources: CL:0000021, GOC:hjd Also known as: female germ-cell nucleus Relationships: is a type of germ cell nucleus [GO:0043073]